{
  "gene": "UniProtKB:Q86XE5",
  "gene_name": "4-hydroxy-2-oxoglutarate aldolase, mitochondrial",
  "gene_symbol": "HOGA1",
  "term_id": "GO:0009436",
  "term_label": "glyoxylate catabolic process"
}